{
  "term_label": "triglyceride homeostasis",
  "gene_name": "Apolipoprotein C-IV",
  "gene_symbol": "APOC4",
  "term_id": "GO:0070328",
  "gene": "UniProtKB:P55056"
}